{
  "gene": "UniProtKB:Q15041",
  "term_id": "GO:0005784",
  "gene_symbol": "ARL6IP1",
  "gene_name": "ADP-ribosylation factor-like protein 6-interacting protein 1",
  "term_label": "Sec61 translocon complex"
}